{
  "term_label": "positive regulation of sensory perception of pain",
  "term_id": "GO:1904058",
  "gene": "UniProtKB:Q6P4H8",
  "gene_name": "ATP synthase subunit C lysine N-methyltransferase",
  "gene_symbol": "ATPSCKMT"
}